{
  "gene": "UniProtKB:Q99547",
  "term_label": "Unknown cellular component",
  "gene_name": "M-phase phosphoprotein 6",
  "gene_symbol": "MPHOSPH6",
  "term_id": "UNKNOWN:0003"
}